{
  "gene_name": "ATP-dependent RNA helicase DDX50",
  "term_label": "RNA helicase activity",
  "term_id": "GO:0003724",
  "gene": "UniProtKB:Q9BQ39",
  "gene_symbol": "DDX50"
}